{
  "gene_symbol": "ENPP6",
  "gene_name": "Glycerophosphocholine cholinephosphodiesterase ENPP6",
  "gene": "UniProtKB:Q6UWR7",
  "term_label": "choline metabolic process",
  "term_id": "GO:0019695"
}